response to non-ionic osmotic stress [GO:0010335] (biological process) Subtypes: cellular response to non-ionic osmotic stress [GO:0071471] Definition: Any process that results in a change in state or activity of a cell or an organism (in terms of movement, secretion, enzyme production, gene expression, etc.) as a result of a stimulus indicating an increase or decrease in the concentration of non-ionic solutes (e.g. mannitol, sorbitol) in the environment. Relationships: is a type of response to osmotic stress [GO:0006970] Sources: GOC:tair_curators